{
  "gene": "UniProtKB:Q16581",
  "term_id": "GO:0007204",
  "gene_symbol": "C3AR1",
  "gene_name": "C3a anaphylatoxin chemotactic receptor",
  "term_label": "positive regulation of cytosolic calcium ion concentration"
}